{
  "term_label": "signaling receptor complex adaptor activity",
  "gene": "UniProtKB:P16520",
  "term_id": "GO:0030159",
  "gene_symbol": "GNB3",
  "gene_name": "Guanine nucleotide-binding protein G(I)_G(S)_G(T) subunit beta-3"
}